{
  "term_label": "negative regulation of membrane protein ectodomain proteolysis",
  "gene": "UniProtKB:P35625",
  "term_id": "GO:0051045",
  "gene_symbol": "TIMP3",
  "gene_name": "Metalloproteinase inhibitor 3"
}